{
  "gene_name": "Lysophospholipid acyltransferase 5",
  "term_label": "1-acylglycerophosphocholine O-acyltransferase activity",
  "gene": "UniProtKB:Q6P1A2",
  "term_id": "GO:0047184",
  "gene_symbol": "LPCAT3"
}